{
  "gene": "UniProtKB:Q9H9Y2",
  "gene_symbol": "RPF1",
  "gene_name": "Ribosome production factor 1",
  "term_label": "maturation of 5.8S rRNA",
  "term_id": "GO:0000460"
}